{
  "term_id": "GO:0000981",
  "term_label": "DNA-binding transcription factor activity, RNA polymerase II-specific",
  "gene_name": "Friend leukemia integration 1 transcription factor",
  "gene_symbol": "FLI1",
  "gene": "UniProtKB:Q01543"
}